PR-toxin biosynthetic process [GO:0140875] (BP) Definition: The chemical reactions and pathways resulting in the formation of PR-toxin, a bicyclic sesquiterpene belonging to the eremophilane class and acting as a mycotoxin. References: PMID:24239699, PMID:27921136 Also known as: PR-toxin anabolism, PR-toxin biosynthesis, PR-toxin formation, PR-toxin synthesis Relationships: is a type of GO:0016106; is a type of GO:0043386